insulin processing [GO:0030070] (biological process) Definition: The formation of mature insulin by proteolysis of the precursor preproinsulin. The signal sequence is first cleaved from preproinsulin to form proinsulin; proinsulin is then cleaved to release the C peptide, leaving the A and B chains of mature insulin linked by disulfide bridges. Sources: ISBN:0198506732 Relationships: is a type of peptide hormone processing [GO:0016486]; is a type of insulin metabolic process [GO:1901142]